{
  "gene_symbol": "IL16",
  "gene_name": "Pro-interleukin-16",
  "gene": "UniProtKB:Q14005",
  "term_id": "GO:0050729",
  "term_label": "positive regulation of inflammatory response"
}